{
  "gene_symbol": "ABCC9",
  "gene": "UniProtKB:O60706",
  "term_id": "GO:0005886",
  "gene_name": "ATP-binding cassette sub-family C member 9",
  "term_label": "plasma membrane"
}